positive regulation of cell differentiation [GO:0045597] (biological process) Definition: Any process that activates or increases the frequency, rate or extent of cell differentiation. Subtypes: GO:0010455, GO:0010718, positive regulation of cell development [GO:0010720], GO:0010744, positive regulation of epithelial cell differentiation [GO:0030858], positive regulation of sorocarp stalk cell differentiation [GO:0031287], positive regulation of chondrocyte differentiation [GO:0032332], GO:0045600, positive regulation of hemocyte differentiation [GO:0045612], positive regulation of myeloid cell differentiation [GO:0045639], positive regulation of myoblast differentiation [GO:0045663], GO:0045666, positive regulation of osteoblast differentiation [GO:0045669], GO:0045690, positive regulation of embryo sac central cell differentiation [GO:0045693], positive regulation of embryo sac egg cell differentiation [GO:0045696], GO:0045699, positive regulation of spermatid nuclear differentiation [GO:0045702], GO:0048336, positive regulation of pigment cell differentiation [GO:0050942], positive regulation of muscle cell differentiation [GO:0051149], positive regulation of cardiac endothelial to mesenchymal transition [GO:0062000], positive regulation of sorocarp spore cell differentiation [GO:1901263], positive regulation of hematopoietic progenitor cell differentiation [GO:1901534], positive regulation of endodermal cell differentiation [GO:1903226], positive regulation of transdifferentiation [GO:1903620], positive regulation of plant epidermal cell differentiation [GO:1903890], positive regulation of sclerenchyma cell differentiation [GO:1904369], GO:1904762, positive regulation of cardiocyte differentiation [GO:1905209], positive regulation of mesodermal cell differentiation [GO:1905772], positive regulation of cell differentiation involved in phenotypic switching [GO:1905917], positive regulation of metanephric DCT cell differentiation [GO:2000594], positive regulation of stem cell differentiation [GO:2000738], positive regulation of skeletal muscle cell differentiation [GO:2001016], positive regulation of tendon cell differentiation [GO:2001051], positive regulation of vasculogenesis [GO:2001214] Relationships: is a type of GO:0045595; is a type of GO:0048522; is_a GO:0051094; positively regulates cell differentiation [GO:0030154] Also known as: up regulation of cell differentiation, up-regulation of cell differentiation, upregulation of cell differentiation, activation of cell differentiation, stimulation of cell differentiation Sources: GOC:go_curators